{
  "term_id": "UNKNOWN:0001",
  "gene_name": "Heparan-alpha-glucosaminide N-acetyltransferase",
  "gene": "UniProtKB:Q68CP4",
  "gene_symbol": "HGSNAT",
  "term_label": "Unknown molecular function"
}